ABC-type fatty-acyl-CoA transporter activity [GO:0015607] (molecular function) Sources: RHEA:15181 Definition: Catalysis of the reaction ATP + H2O + fatty acyl CoA(Side 1) = ADP + phosphate + fatty acyl CoA(Side 2). A fatty acyl CoA group is any acyl group derived from a fatty acid with a coenzyme A group attached to it. Relationships: is a type of organophosphate ester transmembrane transporter activity [GO:0015605]; is a type of nucleobase-containing compound transmembrane transporter activity [GO:0015932]; is a type of ATPase-coupled lipid transmembrane transporter activity [GO:0034040]; is a type of GO:0042887; is a type of GO:0140359; is a type of sulfur compound transmembrane transporter activity [GO:1901682]; is part of fatty-acyl-CoA transport [GO:0015916] Also known as: fatty-acyl-CoA transmembrane transporter activity, ABC-type fatty-acyl-CoA transporter, ATPase-coupled fatty-acyl-CoA transmembrane transporter activity, fatty acyl CoA transporter activity, fatty-acyl-CoA-transporting ATPase